{
  "gene_name": "Sulfotransferase 1A3",
  "gene_symbol": "SULT1A3",
  "term_label": "sulfation",
  "gene": "UniProtKB:P0DMM9",
  "term_id": "GO:0051923"
}